{
  "term_label": "Unknown biological process",
  "term_id": "UNKNOWN:0002",
  "gene": "UniProtKB:Q9BWC9",
  "gene_name": "Coiled-coil domain-containing protein 106",
  "gene_symbol": "CCDC106"
}